{
  "gene_symbol": "A8MVM7",
  "term_id": "UNKNOWN:0003",
  "term_label": "Unknown cellular component",
  "gene_name": "Putative uncharacterized protein ENSP00000382790",
  "gene": "UniProtKB:A8MVM7"
}